{
  "term_id": "GO:0042393",
  "gene_name": "Putative testis-specific Y-encoded-like protein 3",
  "gene": "UniProtKB:Q9H489",
  "gene_symbol": "TSPY26P",
  "term_label": "histone binding"
}